{
  "gene_name": "H_ACA ribonucleoprotein complex subunit 3",
  "gene_symbol": "NOP10",
  "term_label": "telomerase RNA binding",
  "gene": "UniProtKB:Q9NPE3",
  "term_id": "GO:0070034"
}